{
  "gene": "UniProtKB:Q9Y3D6",
  "term_label": "mitochondrial outer membrane",
  "gene_symbol": "FIS1",
  "gene_name": "Mitochondrial fission 1 protein",
  "term_id": "GO:0005741"
}